N-acetylgalactosamine transmembrane transporter activity [GO:0015571] (molecular function) Sources: GOC:ai, GOC:mtg_transport, ISBN:0815340729 Also known as: N-acetylgalactosamine permease activity Definition: Enables the transfer of N-acetylgalactosamine from one side of a membrane to the other. N-acetylgalactosamine, 2-acetamido-2-deoxygalactopyranose, is the n-acetyl derivative of galactosamine. Relationships: is a type of galactosamine transmembrane transporter activity [GO:0019196]; is part of N-acetylgalactosamine transport [GO:0015763] Subtypes: GO:0022881